mesonephric podocyte development [GO:0061257] (biological process) Definition: The process whose specific outcome is the progression of a mesonephric glomerular visceral epithelial cell over time, from its formation to the mature structure. A mesonephric glomerular visceral epithelial cell is a specialized epithelial cell that contains 'feet' that interdigitate with the 'feet' of other glomerular epithelial cells in the mesonephros. Sources: GOC:mtg_kidney_jan10 Also known as: mesonephric glomerular visceral epithelial cell development Relationships: is a type of mesonephric glomerular epithelial cell development [GO:0061251]; is_a GO:0072015; is part of mesonephric podocyte differentiation [GO:0061256]